nephron tubule epithelial cell differentiation [GO:0072160] (biological process) Sources: GOC:mtg_kidney_jan10 Relationships: is a type of epithelial cell differentiation involved in kidney development [GO:0035850]; is part of GO:0072080 Definition: The process in which relatively unspecialized cells acquire specialized structural and/or functional features that characterize the cells of the nephron tubule as it progresses from its formation to the mature state. Subtypes: pronephric nephron tubule epithelial cell differentiation [GO:0035778], mesonephric nephron tubule epithelial cell differentiation [GO:0061265], metanephric nephron tubule epithelial cell differentiation [GO:0072257] Regulation: regulated by regulation of nephron tubule epithelial cell differentiation [GO:0072182]; negatively regulated by negative regulation of nephron tubule epithelial cell differentiation [GO:0072183]; positively regulated by positive regulation of nephron tubule epithelial cell differentiation [GO:2000768]